{
  "gene": "UniProtKB:P49913",
  "gene_name": "Cathelicidin antimicrobial peptide",
  "term_id": "GO:0005615",
  "gene_symbol": "CAMP",
  "term_label": "extracellular space"
}